{
  "gene": "UniProtKB:Q16609",
  "gene_name": "Putative apolipoprotein(a)-like protein 2",
  "term_id": "UNKNOWN:0002",
  "term_label": "Unknown biological process",
  "gene_symbol": "LPAL2"
}